{
  "gene_symbol": "DYNLT4",
  "gene_name": "Dynein light chain Tctex-type 4",
  "term_id": "GO:0007018",
  "term_label": "microtubule-based movement",
  "gene": "UniProtKB:Q5JR98"
}